{
  "term_label": "positive regulation of T cell mediated cytotoxicity",
  "gene": "UniProtKB:P10321",
  "term_id": "GO:0001916",
  "gene_name": "HLA class I histocompatibility antigen, C alpha chain",
  "gene_symbol": "HLA-C"
}